{
  "term_label": "DNA-binding transcription activator activity, RNA polymerase II-specific",
  "gene": "UniProtKB:A6NDR6",
  "term_id": "GO:0001228",
  "gene_symbol": "MEIS3P1",
  "gene_name": "Putative homeobox protein Meis3-like 1"
}